positive regulation of nodal signaling pathway [GO:0141092] (biological process) Definition: Any process that increases the rate, frequency or extent of nodal signaling pathway. References: PMID:17239842 Relationships: is a type of GO:0032927; is a type of regulation of nodal signaling pathway [GO:1900107]; positively regulates nodal signaling pathway [GO:0038092]